{
  "gene_symbol": "TRAJ37",
  "gene_name": "T cell receptor alpha joining 37 (Fragment)",
  "gene": "UniProtKB:A0A087X096",
  "term_id": "UNKNOWN:0002",
  "term_label": "Unknown biological process"
}